{
  "term_label": "mRNA binding",
  "gene": "UniProtKB:Q14966",
  "gene_symbol": "ZNF638",
  "term_id": "GO:0003729",
  "gene_name": "Zinc finger protein 638"
}